{
  "term_label": "G protein-coupled receptor signaling pathway, coupled to cyclic nucleotide second messenger",
  "gene_symbol": "HTR4",
  "gene_name": "5-hydroxytryptamine receptor 4",
  "gene": "UniProtKB:Q13639",
  "term_id": "GO:0007187"
}